{
  "gene_name": "Interferon-induced, double-stranded RNA-activated protein kinase",
  "term_id": "GO:0005634",
  "gene_symbol": "EIF2AK2",
  "gene": "UniProtKB:P19525",
  "term_label": "nucleus"
}